{
  "term_label": "chromatin remodeling",
  "gene_name": "Chromodomain-helicase-DNA-binding protein 8",
  "gene_symbol": "CHD8",
  "term_id": "GO:0006338",
  "gene": "UniProtKB:Q9HCK8"
}